{
  "gene_name": "Protein disulfide-isomerase-like protein of the testis",
  "term_id": "UNKNOWN:0001",
  "term_label": "Unknown molecular function",
  "gene": "UniProtKB:Q8N807",
  "gene_symbol": "PDILT"
}